{
  "term_id": "GO:0032956",
  "term_label": "regulation of actin cytoskeleton organization",
  "gene_symbol": "RHOA",
  "gene": "UniProtKB:P61586",
  "gene_name": "Transforming protein RhoA"
}